response to cadmium ion [GO:0046686] (biological process) Subtypes: GO:0071276, GO:1990170 Definition: Any process that results in a change in state or activity of a cell or an organism (in terms of movement, secretion, enzyme production, gene expression, etc.) as a result of a cadmium (Cd) ion stimulus. Sources: GOC:ai Relationships: is a type of response to metal ion [GO:0010038] Also known as: response to cadmium, cadmium sensitivity/resistance